{
  "term_id": "GO:0048854",
  "gene_name": "F-box_WD repeat-containing protein 11",
  "gene_symbol": "FBXW11",
  "gene": "UniProtKB:Q9UKB1",
  "term_label": "brain morphogenesis"
}